{
  "term_label": "plasma membrane",
  "gene_symbol": "EPHA3",
  "gene_name": "Ephrin type-A receptor 3",
  "term_id": "GO:0005886",
  "gene": "UniProtKB:P29320"
}